stomach development [GO:0062094] (biological process) Relationships: is a type of anatomical structure development [GO:0048856]; is part of GO:0048565 Definition: The process whose specific outcome is the progression of the stomach over time, from its formation to the mature structure. The stomach is an expanded region of the vertebrate alimentary tract that serves as a food storage compartment and digestive organ. References: PMID:11967278